{
  "gene_name": "Fibroblast growth factor 8",
  "gene_symbol": "FGF8",
  "term_id": "GO:0005737",
  "term_label": "cytoplasm",
  "gene": "UniProtKB:P55075"
}